{
  "term_label": "Unknown cellular component",
  "term_id": "UNKNOWN:0003",
  "gene": "UniProtKB:Q53RT3",
  "gene_name": "Retroviral-like aspartic protease 1",
  "gene_symbol": "ASPRV1"
}